{
  "gene": "UniProtKB:Q9H1H9",
  "gene_name": "Kinesin-like protein KIF13A",
  "gene_symbol": "KIF13A",
  "term_label": "cytoplasm",
  "term_id": "GO:0005737"
}